{
  "term_id": "GO:0005856",
  "term_label": "cytoskeleton",
  "gene_symbol": "KANK4",
  "gene_name": "KN motif and ankyrin repeat domain-containing protein 4",
  "gene": "UniProtKB:Q5T7N3"
}